positive regulation of heart rate involved in baroreceptor response to decreased systemic arterial blood pressure [GO:0001988] (biological process) Definition: Any process that activates, maintains or increases the frequency, rate or extent of heart contraction as a result of the baroreceptor response to decreased blood pressure. Relationships: is a type of positive regulation of heart rate [GO:0010460]; is part of baroreceptor response to decreased systemic arterial blood pressure [GO:0001982] Sources: ISBN:0721643949 Also known as: positive control of heart contraction rate in baroreceptor response to decreased blood pressure, positive regulation of cardiac contraction rate in baroreceptor response to decreased blood pressure, up regulation of heart contraction rate in baroreceptor response to decreased blood pressure, up-regulation of heart contraction rate in baroreceptor response to decreased blood pressure, upregulation of heart contraction rate in baroreceptor response to decreased blood pressure, activation of heart contraction rate in baroreceptor response to decreased blood pressure, stimulation of heart contraction rate in baroreceptor response to decreased blood pressure, positive regulation of heart contraction rate in baroreceptor response to decreased blood pressure